{
  "gene_symbol": "A0A5F9ZH88",
  "gene_name": "Immunoglobulin subtype domain-containing protein",
  "gene": "UniProtKB:A0A5F9ZH88",
  "term_label": "immune response-inhibiting cell surface receptor signaling pathway",
  "term_id": "GO:0002767"
}